cholate-CoA ligase activity [GO:0047747] (molecular function) Also known as: 3-alpha,7-alpha,12-alpha-trihydroxy-5-beta-cholestanate-CoA ligase activity, 3-alpha,7-alpha,12-alpha-trihydroxy-5-beta-cholestanate--CoA ligase activity, 3-alpha,7-alpha,12-alpha-trihydroxy-5-beta-cholestanate:CoA ligase (AMP-forming) activity, 3-alpha,7-alpha,12-alpha-trihydroxy-5-beta-cholestanoate-CoA ligase activity, 3-alpha,7-alpha,12-alpha-trihydroxy-5-beta-cholestanoate-CoA synthetase activity, 3-alpha,7-alpha,12-alpha-trihydroxy-5-beta-cholestanoyl coenzyme A synthetase activity, 3alpha,7alpha,12alpha-trihydroxy-5beta-cholestanate-CoA ligase activity, 3alpha,7alpha,12alpha-trihydroxy-5beta-cholestanate:CoA ligase (AMP-forming), 3alpha,7alpha,12alpha-trihydroxy-5beta-cholestanoate-CoA ligase activity, 3alpha,7alpha,12alpha-trihydroxy-5beta-cholestanoate-CoA synthetase activity, 3alpha,7alpha,12alpha-trihydroxy-5beta-cholestanoyl coenzyme A synthetase activity, BAL activity, THCA-CoA ligase activity, bile acid CoA ligase activity, bile acid coenzyme A ligase activity, cholate thiokinase activity, cholate:CoA ligase (AMP-forming), cholic acid:CoA ligase activity, cholic thiokinase activity, choloyl coenzyme A synthetase activity, choloyl-CoA synthetase activity, cholyl-CoA synthetase activity, trihydroxycoprostanoyl-CoA synthetase activity Relationships: is a type of CoA-ligase activity [GO:0016405]; is a type of acid-thiol ligase activity [GO:0016878] Sources: EC:6.2.1.7 Definition: Catalysis of the reactions: (1) ATP + cholate + CoA = AMP + diphosphate + choloyl-CoA and (2) ATP + (25R)-3alpha,7alpha,12alpha-trihydroxy-5beta-cholestan-26-oate + CoA = AMP + diphosphate + (25R)-3alpha,7alpha,12alpha-trihydroxy-5beta-cholestanoyl-CoA. This reaction is the first step in the conjugation of bile acids with amino acids, converting bile acids into their acyl-CoA thioesters. Chenodeoxycholate, deoxycholate, lithocholate and trihydroxycoprostanoate can also act as substrates.